{
  "gene_name": "Olfactory receptor 2T29",
  "term_id": "GO:0004984",
  "gene": "UniProtKB:Q8NH02",
  "gene_symbol": "OR2T29",
  "term_label": "olfactory receptor activity"
}